{
  "gene_name": "Plexin-A1",
  "term_label": "synapse assembly",
  "term_id": "GO:0007416",
  "gene": "UniProtKB:Q9UIW2",
  "gene_symbol": "PLXNA1"
}